{
  "gene_name": "Protein-lysine 6-oxidase",
  "gene_symbol": "LOX",
  "gene": "UniProtKB:P28300",
  "term_id": "GO:0035791",
  "term_label": "platelet-derived growth factor receptor-beta signaling pathway"
}